positive regulation of cutin biosynthetic process [GO:1901959] (biological process) Definition: Any process that activates or increases the frequency, rate or extent of cutin biosynthetic process. References: PMID:23243127 Sources: GOC:TermGenie, GOC:tb Also known as: activation of cutin anabolism, activation of cutin biosynthesis, activation of cutin formation, activation of cutin synthesis, positive regulation of cutin anabolism, positive regulation of cutin biosynthesis, positive regulation of cutin formation, positive regulation of cutin synthesis, up regulation of cutin anabolism, up regulation of cutin biosynthesis, up regulation of cutin biosynthetic process, up regulation of cutin formation, up regulation of cutin synthesis, up-regulation of cutin anabolism, up-regulation of cutin biosynthesis, up-regulation of cutin biosynthetic process, up-regulation of cutin formation, up-regulation of cutin synthesis, upregulation of cutin anabolism, upregulation of cutin biosynthesis, upregulation of cutin biosynthetic process, upregulation of cutin formation, upregulation of cutin synthesis, activation of cutin biosynthetic process Relationships: is a type of positive regulation of macromolecule biosynthetic process [GO:0010557]; is a type of GO:1901957; positively regulates cutin biosynthetic process [GO:0010143]